regulation of collecting lymphatic vessel constriction [GO:1903814] (biological process) Definition: Any process that modulates the frequency, rate or extent of collecting lymphatic vessel constriction. References: PMID:23897233 Sources: GOC:TermGenie, GO_REF:0000058 Also known as: regulation of lymphatic vessel myogenic constriction Relationships: is a type of regulation of system process [GO:0044057]; is a type of regulation of anatomical structure size [GO:0090066]; regulates collecting lymphatic vessel constriction [GO:1990192] Subtypes: GO:1903815, positive regulation of collecting lymphatic vessel constriction [GO:1903816]